{
  "gene_symbol": "KLHL23",
  "term_label": "ubiquitin-like ligase-substrate adaptor activity",
  "term_id": "GO:1990756",
  "gene": "UniProtKB:Q8NBE8",
  "gene_name": "Kelch-like protein 23"
}